cytosolic proteasome regulatory particle, base subcomplex [GO:0031612] (cellular component) Definition: The subcomplex of the proteasome regulatory particle that directly associates with the proteasome core complex located in the cytosol of the cell. Sources: GOC:mah, GOC:mtg_sensu Relationships: is a type of GO:0008540; is part of cytosolic proteasome regulatory particle [GO:0031600]